{
  "term_label": "Unknown biological process",
  "gene_symbol": "MKKS",
  "gene_name": "MKKS centrosomal shuttling protein",
  "term_id": "UNKNOWN:0002",
  "gene": "UniProtKB:V9GZ13"
}